pituitary adenylate cyclase-activating polypeptide receptor activity [GO:0001634] (molecular function) Relationships: is_a GO:0004930 Definition: A G protein-coupled receptor that interacts with pituitary adenylate cyclase-activating polypeptide. Sources: GOC:dph, GOC:tb Also known as: PACAP receptor, pituitary adenylate cyclase activating polypeptide receptor, pituitary adenylate cyclase activating protein receptor activity, pituitary adenylyl cyclase activating protein receptor activity, pituitary adenylate cyclase-activating peptide receptor activity